{
  "term_id": "GO:0010468",
  "gene": "UniProtKB:A0A3B3IT33",
  "gene_symbol": "TRIM51G",
  "gene_name": "Putative tripartite motif-containing protein 51G",
  "term_label": "regulation of gene expression"
}